{
  "gene": "UniProtKB:A6NGS2",
  "gene_symbol": "ERICH4",
  "gene_name": "Glutamate-rich protein 4",
  "term_id": "UNKNOWN:0003",
  "term_label": "Unknown cellular component"
}